aminoglycoside 6-kinase activity [GO:0050300] (molecular function) Also known as: ATP:streptomycin 6-phosphotransferase activity, SM 6-kinase activity, streptidine kinase (phosphorylating), streptidine kinase activity, streptomycin 6-O-phosphotransferase activity, streptomycin 6-kinase (phosphorylating), streptomycin 6-kinase activity, streptomycin 6-phosphotransferase activity, APH(6) activity Relationships: is a type of aminoglycoside phosphotransferase activity [GO:0034071] Definition: Catalysis of the reaction: ATP + streptomycin = ADP + 2 H+ + streptomycin 6-phosphate. Sources: EC:2.7.1.72, RHEA:22268